{
  "gene_symbol": "A0A7P0T9M0",
  "term_label": "Unknown biological process",
  "gene": "UniProtKB:A0A7P0T9M0",
  "gene_name": "Uncharacterized protein",
  "term_id": "UNKNOWN:0002"
}